{
  "gene_name": "Olfactory receptor",
  "gene_symbol": "LOC124905359",
  "term_id": "GO:0004984",
  "gene": "UniProtKB:A0A0G2JNH3",
  "term_label": "olfactory receptor activity"
}